{
  "gene_name": "Ephrin type-B receptor 4",
  "gene_symbol": "EPHB4",
  "gene": "UniProtKB:P54760",
  "term_label": "ephrin receptor signaling pathway",
  "term_id": "GO:0048013"
}